{
  "gene_name": "Pyrroline-5-carboxylate reductase 1, mitochondrial",
  "term_label": "pyrroline-5-carboxylate reductase activity",
  "gene_symbol": "PYCR1",
  "term_id": "GO:0004735",
  "gene": "UniProtKB:P32322"
}